{
  "gene_name": "Kinesin-like protein KIF2B",
  "gene_symbol": "KIF2B",
  "gene": "UniProtKB:Q8N4N8",
  "term_id": "GO:0003777",
  "term_label": "microtubule motor activity"
}